{
  "term_id": "GO:0005634",
  "term_label": "nucleus",
  "gene_symbol": "HESX1",
  "gene_name": "Homeobox expressed in ES cells 1",
  "gene": "UniProtKB:Q9UBX0"
}